{
  "term_label": "nucleosome",
  "gene_name": "Histone H2B type 1-L",
  "gene_symbol": "H2BC13",
  "gene": "UniProtKB:Q99880",
  "term_id": "GO:0000786"
}